{
  "gene_name": "Dual specificity mitogen-activated protein kinase kinase 4",
  "gene_symbol": "MAP2K4",
  "term_id": "UNKNOWN:0003",
  "term_label": "Unknown cellular component",
  "gene": "UniProtKB:P45985"
}